{
  "gene": "UniProtKB:A6NK97",
  "term_label": "Unknown cellular component",
  "term_id": "UNKNOWN:0003",
  "gene_symbol": "SLC22A20P",
  "gene_name": "Solute carrier family 22 member 20"
}